{
  "term_id": "GO:0016020",
  "gene": "UniProtKB:Q9BV23",
  "gene_name": "Monoacylglycerol lipase ABHD6",
  "term_label": "membrane",
  "gene_symbol": "ABHD6"
}